{
  "gene": "UniProtKB:Q13868",
  "term_label": "poly(A)-dependent snoRNA 3'-end processing",
  "gene_symbol": "EXOSC2",
  "gene_name": "Exosome complex component RRP4",
  "term_id": "GO:0071051"
}